negative regulation of chemokine (C-X-C motif) ligand 9 production [GO:0035395] (biological process) Also known as: negative regulation of CXCL9 production, negative regulation of MIG production Definition: Any process that stops, prevents, or reduces the frequency, rate, or extent of production of chemokine (C-X-C motif) ligand 9. Relationships: is a type of negative regulation of chemokine production [GO:0032682]; is a type of GO:0035394; negatively regulates chemokine (C-X-C motif) ligand 9 production [GO:0035393] Sources: GOC:bf